{
  "gene_symbol": "ATG5",
  "gene_name": "Autophagy protein 5",
  "term_label": "autophagosome",
  "term_id": "GO:0005776",
  "gene": "UniProtKB:Q9H1Y0"
}